{
  "gene_name": "Calcitonin receptor",
  "gene_symbol": "CALCR",
  "term_label": "adenylate cyclase-activating G protein-coupled receptor signaling pathway",
  "gene": "UniProtKB:P30988",
  "term_id": "GO:0007189"
}